nipple sheath formation [GO:0060659] (biological process) References: PMID:12558599 Sources: GOC:dph Relationships: is a type of anatomical structure formation involved in morphogenesis [GO:0048646]; is part of nipple morphogenesis [GO:0060658] Definition: The developmental process pertaining to the initial formation of the nipple sheath from the unspecified epidermis. This process begins with a circular ingrowth of the epidermis around the region of the mammary sprout. It ends before the region begins to elevate.